{
  "gene_symbol": "ULK3",
  "gene": "UniProtKB:Q6PHR2",
  "gene_name": "Serine_threonine-protein kinase ULK3",
  "term_id": "GO:0042594",
  "term_label": "response to starvation"
}